{
  "gene_name": "Storkhead-box protein 1",
  "term_id": "GO:0005634",
  "gene_symbol": "STOX1",
  "term_label": "nucleus",
  "gene": "UniProtKB:Q6ZVD7"
}